heterochromatin boundary formation [GO:0033696] (biological process) Definition: A process that forms a boundary that limits the spreading of heterochromatin along a chromosome. Also known as: regulation of extent of heterochromatin formation, maintenance of heterochromatin boundaries, negative regulation of extent of heterochromatin assembly, negative regulation of extent of heterochromatin formation, negative regulation of heterochromatin spreading, regulation of extent of heterochromatin assembly, regulation of heterochromatin spreading Sources: GOC:mah Relationships: is a type of heterochromatin organization [GO:0070828]; is part of GO:0031507